positive regulation of mitochondrial fission [GO:0090141] (biological process) Also known as: positive regulation of mitochondrial division Definition: Any process that increases the rate, frequency or extent of mitochondrial fission. Mitochondrial fission is the division of a mitochondrion within a cell to form two or more separate mitochondrial compartments. Sources: GOC:ascb_2009, GOC:dph, GOC:tb Relationships: is_a GO:0010638; is a type of positive regulation of developmental process [GO:0051094]; is_a GO:0090140; positively regulates mitochondrial fission [GO:0000266]